{
  "gene_symbol": "HMSD",
  "gene_name": "Serpin-like protein HMSD",
  "term_label": "Unknown biological process",
  "term_id": "UNKNOWN:0002",
  "gene": "UniProtKB:A8MTL9"
}